{
  "term_label": "cholesterol efflux",
  "gene_symbol": "ABCG4",
  "term_id": "GO:0033344",
  "gene": "UniProtKB:Q9H172",
  "gene_name": "ATP-binding cassette sub-family G member 4"
}